branched-chain amino acid catabolic process to carboxylic acid via Ehrlich pathway [GO:0000953] (biological process) Definition: The chemical reactions and pathways involving the catabolism of amino acids to produce carboxylic acids with one carbon less than the starting amino acid. In S. cerevisiae, this is known to occur for leucine, isoleucine, valine, methionine, phenylalanine, tyrosine, or tryptophan. When a branched chain family amino acid, leucine, isoleucine, or valine, is used as the substrate, 3-methylbutanoate, 2-methylbutanoate, or 2-methylpropanoate, respectively, is produced. Often referred to as the Ehrlich pathway, these reactions generally occur during fermentation to produce a variety of carboxylic acids, sometimes collectively referred to as fusel acids. Depending on the redox state of the cells, alcohol derivatives may be produced instead of carboxylic acids. References: PMID:18281432 Sources: GOC:krc Also known as: branched chain family amino acid catabolic process to carboxylic acid via Ehrlich pathway Relationships: is a type of amino acid catabolic process to carboxylic acid via Ehrlich pathway [GO:0000948]; is a type of branched-chain amino acid catabolic process [GO:0009083]